{
  "term_id": "GO:0000976",
  "gene_name": "Zinc finger protein 268",
  "gene": "UniProtKB:Q14587",
  "term_label": "transcription cis-regulatory region binding",
  "gene_symbol": "ZNF268"
}